{
  "term_label": "chromatin binding",
  "gene_name": "Double-strand-break repair protein rad21-like protein 1",
  "term_id": "GO:0003682",
  "gene_symbol": "RAD21L1",
  "gene": "UniProtKB:Q9H4I0"
}